{
  "term_label": "microtubule organizing center",
  "gene": "UniProtKB:Q9P2S5",
  "gene_name": "WD repeat-containing protein WRAP73",
  "gene_symbol": "WRAP73",
  "term_id": "GO:0005815"
}